regulation of enamel mineralization [GO:0070173] (biological process) Relationships: is a type of regulation of tooth mineralization [GO:0070170]; regulates enamel mineralization [GO:0070166] Sources: GOC:BHF, GOC:mah Definition: Any process that modulates the frequency, rate or extent of enamel mineralization, the deposition of calcium salts in tooth enamel. Subtypes: negative regulation of enamel mineralization [GO:0070174], positive regulation of enamel mineralization [GO:0070175]